{
  "term_id": "UNKNOWN:0002",
  "gene_name": "Putative protein PRAC2",
  "term_label": "Unknown biological process",
  "gene_symbol": "PRAC2",
  "gene": "UniProtKB:D3DTV9"
}